{
  "gene_name": "Beta-secretase 1",
  "term_label": "protein processing",
  "gene": "UniProtKB:P56817",
  "gene_symbol": "BACE1",
  "term_id": "GO:0016485"
}